{
  "gene": "UniProtKB:Q6ZTQ4",
  "gene_symbol": "CDHR3",
  "term_id": "GO:0045296",
  "gene_name": "Cadherin-related family member 3",
  "term_label": "cadherin binding"
}